antimicrobial peptide biosynthetic process [GO:0002777] (biological process) Definition: The chemical reactions and pathways resulting in the formation of an antimicrobial peptide. Such peptides may have protective properties against bacteria, fungi, viruses, or protozoa. Regulation: regulated by GO:0002805; negatively regulated by negative regulation of antimicrobial peptide biosynthetic process [GO:0002806]; positively regulated by positive regulation of antimicrobial peptide biosynthetic process [GO:0002807] Relationships: is a type of GO:0043043; is part of antimicrobial peptide production [GO:0002775] References: PMID:11807545, PMID:15638771 Sources: GOC:add, ISBN:0781735149 Subtypes: antibacterial peptide biosynthetic process [GO:0002780], GO:0002783